vitamin D receptor signaling pathway [GO:0070561] (biological process) References: PMID:12637589 Sources: GOC:BHF, GOC:mah Also known as: VDR signaling pathway, intracellular vitamin D receptor signaling pathway, nuclear receptor-mediated vitamin D signaling pathway, vitamin D receptor signalling pathway, calcitriol signaling pathway Definition: A nuclear receptor-mediated signaling pathway initiated by vitamin D binding to an intracellular receptor of the nuclear receptor protein family, and ending with regulation of a downstream cellular process, e.g. transcription. Regulation: regulated by GO:0070562; negatively regulated by negative regulation of vitamin D receptor signaling pathway [GO:0070563]; positively regulated by positive regulation of vitamin D receptor signaling pathway [GO:0070564] Relationships: is a type of GO:0009755; is a type of nuclear receptor-mediated signaling pathway [GO:0141193]; is part of cellular response to vitamin D [GO:0071305]